{
  "gene_symbol": "CXCL9",
  "term_id": "GO:0071222",
  "term_label": "cellular response to lipopolysaccharide",
  "gene_name": "C-X-C motif chemokine 9",
  "gene": "UniProtKB:Q07325"
}